{
  "gene_name": "Uncharacterized protein encoded by LINC01547",
  "gene_symbol": "LINC01547",
  "gene": "UniProtKB:P58512",
  "term_label": "Unknown molecular function",
  "term_id": "UNKNOWN:0001"
}